{
  "term_label": "collagen fibril organization",
  "gene_name": "Collagen alpha-2(I) chain",
  "gene": "UniProtKB:P08123",
  "term_id": "GO:0030199",
  "gene_symbol": "COL1A2"
}